negative regulation of filamentous growth of a population of unicellular organisms in response to biotic stimulus [GO:1900444] (biological process) Also known as: down regulation of filamentous growth of a population of unicellular organisms in response to biotic stimulus, down-regulation of filamentous growth of a population of unicellular organisms in response to biotic stimulus, downregulation of filamentous growth of a population of unicellular organisms in response to biotic stimulus, inhibition of filamentous growth of a population of unicellular organisms in response to biotic stimulus Relationships: is a type of negative regulation of response to biotic stimulus [GO:0002832]; is a type of negative regulation of filamentous growth of a population of unicellular organisms [GO:1900429]; is a type of GO:1900443; negatively regulates filamentous growth of a population of unicellular organisms in response to biotic stimulus [GO:0036180] Definition: Any process that stops, prevents or reduces the frequency, rate or extent of filamentous growth of a population of unicellular organisms in response to biotic stimulus. Sources: GOC:TermGenie, GOC:di